fatty acid omega-hydroxylase activity [GO:0120250] (molecular function) Definition: Catalysis of the reaction: an omega-methyl fatty acid + O2 + reduced [NADPH--hemoprotein reductase] = an omega-hydroxy fatty acid + H+ + H2O + oxidized [NADPH--hemoprotein reductase]. Relationships: is a type of oxidoreductase activity, acting on paired donors, with incorporation or reduction of molecular oxygen, reduced flavin or flavoprotein as one donor, and incorporation of one atom of oxygen [GO:0016712] Sources: GOC:krc, RHEA:39023 Also known as: omega-hydroxylase activity Subtypes: long-chain fatty acid omega-hydroxylase activity [GO:0102033], very long-chain fatty acid omega-hydroxylase activity [GO:0140692], medium-chain fatty acid omega-hydroxylase activity [GO:0140981]